G protein-coupled opsin signaling pathway [GO:0016056] (biological process) Definition: A G protein-coupled receptor signaling pathway that starts with an opsin being activated by a photon, and ending with the light signal being trasmitted through the synapses. The signal can be transmitted via different Galpha subunits types: Go, Gs, Gq, and Gt. Subtypes: phospholipase C-activating opsin-mediated signaling pathway [GO:0030265], GO:0141190 Regulation: negatively regulated by negative regulation of opsin-mediated signaling pathway [GO:0016059]; regulated by regulation of opsin-mediated signaling pathway [GO:0022400] References: PMID:19720651, PMID:36272560 Sources: GOC:bf, GOC:dph, GOC:hb, GOC:signaling, GOC:tb Relationships: is a type of G protein-coupled receptor signaling pathway [GO:0007186]; is a type of phototransduction [GO:0007602]; is a type of cellular response to light stimulus [GO:0071482]; is part of phototransduction, visible light [GO:0007603] Also known as: rhodopsin mediated signaling pathway, G protein-mediated opsin signaling pathway, rhodopsin mediated phototransduction, rhodopsin mediated signalling pathway, rhodopsin signaling